{
  "gene": "UniProtKB:P54920",
  "gene_symbol": "NAPA",
  "term_label": "synaptobrevin 2-SNAP-25-syntaxin-1a complex",
  "term_id": "GO:0070044",
  "gene_name": "Alpha-soluble NSF attachment protein"
}